{
  "gene": "UniProtKB:Q9H173",
  "term_label": "adenyl-nucleotide exchange factor activity",
  "term_id": "GO:0000774",
  "gene_symbol": "SIL1",
  "gene_name": "Nucleotide exchange factor SIL1"
}